snRNA stem-loop binding [GO:0035614] (molecular function) References: PMID:16568238, PMID:20455544 Sources: GOC:sart Relationships: is_a snRNA binding [GO:0017069]; is a type of RNA stem-loop binding [GO:0035613] Also known as: small nuclear RNA stem-loop binding, snRNA hairpin binding, snRNA hairpin loop binding Definition: Binding to a stem-loop in a small nuclear RNA (snRNA). An RNA stem-loop is a secondary RNA structure consisting of a double-stranded RNA (dsRNA) stem and a terminal loop.